Rad6-Rad18 complex [GO:0097505] (cellular component) Definition: A ubiquitin ligase complex found to be involved in post-replicative bypass of UV-damaged DNA and UV mutagenesis. In S. cerevisiae, the complex contains the ubiquitin conjugating enzyme Rad6 and Rad18, a protein containing a RING finger motif and a nucleotide binding motif. The yeast Rad6-Rad18 heterodimer has ubiquitin conjugating activity, binds single-stranded DNA, and possesses single-stranded DNA-dependent ATPase activity. References: PMID:9287349 Sources: GOC:jd Relationships: is a type of ubiquitin ligase complex [GO:0000151]